{
  "term_label": "nucleoplasm",
  "gene": "UniProtKB:E7EW31",
  "gene_symbol": "PROB1",
  "term_id": "GO:0005654",
  "gene_name": "Proline-rich basic protein 1"
}